lactoylglutathione lyase activity [GO:0004462] (molecular function) Relationships: is a type of carbon-sulfur lyase activity [GO:0016846] Definition: Catalysis of the reaction: (R)-S-lactoylglutathione = glutathione + methylglyoxal. Sources: EC:4.4.1.5, RHEA:19069 Also known as: (R)-S-lactoylglutathione methylglyoxal-lyase (isomerizing) activity, (R)-S-lactoylglutathione methylglyoxal-lyase (isomerizing; glutathione-forming), aldoketomutase activity, glyoxalase I activity, glyoxylase I, ketone-aldehyde mutase activity, methylglyoxalase activity